{
  "gene_name": "Microtubule-associated serine_threonine-protein kinase 1",
  "term_id": "GO:0007010",
  "gene_symbol": "MAST1",
  "term_label": "cytoskeleton organization",
  "gene": "UniProtKB:Q9Y2H9"
}